{
  "gene_name": "ADP-ribosylation factor 1",
  "gene_symbol": "ARF1",
  "term_id": "GO:0005737",
  "gene": "UniProtKB:P84077",
  "term_label": "cytoplasm"
}